{
  "gene": "UniProtKB:Q08ET2",
  "term_label": "plasma membrane",
  "term_id": "GO:0005886",
  "gene_name": "Sialic acid-binding Ig-like lectin 14",
  "gene_symbol": "SIGLEC14"
}